{
  "gene": "UniProtKB:A6NGY5",
  "term_id": "GO:0005886",
  "term_label": "plasma membrane",
  "gene_name": "Olfactory receptor 51F1",
  "gene_symbol": "OR51F1"
}